{
  "gene_symbol": "RAD51",
  "gene": "UniProtKB:Q06609",
  "gene_name": "DNA repair protein RAD51 homolog 1",
  "term_label": "chromosome organization involved in meiotic cell cycle",
  "term_id": "GO:0070192"
}